{
  "gene_symbol": "RNF123",
  "gene": "UniProtKB:Q5XPI4",
  "term_id": "GO:0005737",
  "term_label": "cytoplasm",
  "gene_name": "E3 ubiquitin-protein ligase RNF123"
}